{
  "gene": "UniProtKB:Q9H7L9",
  "term_label": "histone deacetylase binding",
  "gene_name": "Sin3 histone deacetylase corepressor complex component SDS3",
  "gene_symbol": "SUDS3",
  "term_id": "GO:0042826"
}